cellular bud site selection [GO:0000282] (biological process) Definition: The specification of the site where a daughter cell will form, in organisms that reproduce by budding. An example of this process is found in Saccharomyces cerevisiae. Sources: GOC:mah Also known as: bud site selection/establishment of cell polarity Note: Note that this term was split from 'bud site selection/establishment of cell polarity (sensu Saccharomyces) ; GO:0007115' (a sibling term, 'establishment of cell polarity (sensu Saccharomyces) ; GO:0000283', was created but has since been merged with 'establishment of cell polarity' ; GO:0030010). Relationships: is a type of establishment of cell polarity [GO:0030010]; is a type of mitotic cell cycle process [GO:1903047]; is part of mitotic cytokinesis [GO:0000281] Subtypes: axial cellular bud site selection [GO:0007120], GO:0007121